{
  "term_id": "GO:0005739",
  "gene": "UniProtKB:Q2TB90",
  "gene_name": "Hexokinase HKDC1",
  "term_label": "mitochondrion",
  "gene_symbol": "HKDC1"
}